B axonemal microtubule [GO:0097650] (cellular component) Relationships: is a type of axonemal microtubule [GO:0005879]; is part of GO:0097545 Sources: GOC:cilia, ISBN:0716731363 Also known as: B tubule Definition: An incomplete microtubule containing 10 protofilaments that fuses with a complete microtubule called A tubule (containing 13 protofilaments) to form an axonemal outer doublet.